{
  "term_label": "sialic acid binding",
  "gene_symbol": "SIGLEC6",
  "term_id": "GO:0033691",
  "gene": "UniProtKB:O43699",
  "gene_name": "Sialic acid-binding Ig-like lectin 6"
}